{
  "term_label": "ATPase-coupled intramembrane lipid transporter activity",
  "gene_symbol": "ATP8B2",
  "term_id": "GO:0140326",
  "gene": "UniProtKB:P98198",
  "gene_name": "Phospholipid-transporting ATPase ID"
}